{
  "gene_symbol": "OR1E1",
  "gene_name": "Olfactory receptor 1E1",
  "term_id": "GO:0004984",
  "gene": "UniProtKB:P30953",
  "term_label": "olfactory receptor activity"
}